{
  "gene_name": "TOX high mobility group box family member 4",
  "gene": "UniProtKB:O94842",
  "term_label": "chromatin DNA binding",
  "gene_symbol": "TOX4",
  "term_id": "GO:0031490"
}